{
  "term_label": "WASH complex",
  "term_id": "GO:0071203",
  "gene": "UniProtKB:Q2M389",
  "gene_name": "WASH complex subunit 4",
  "gene_symbol": "WASHC4"
}